{
  "term_label": "regulation of Golgi to plasma membrane protein transport",
  "term_id": "GO:0042996",
  "gene_symbol": "VAMP4",
  "gene_name": "Vesicle-associated membrane protein 4",
  "gene": "UniProtKB:O75379"
}